{
  "term_id": "GO:0005829",
  "gene_name": "Ribonucleoside-diphosphate reductase subunit M2 B",
  "gene_symbol": "RRM2B",
  "term_label": "cytosol",
  "gene": "UniProtKB:Q7LG56"
}